negative regulation of monoatomic anion transport [GO:1903792] (BP) References: PMID:11336802 Sources: GOC:TermGenie, GO_REF:0000058 Subtypes: negative regulation of anion transmembrane transport [GO:1903960], negative regulation of iodide transport [GO:1904202], negative regulation of chloride transport [GO:2001226] Also known as: negative regulation of anion transport, down regulation of anion transport, down-regulation of anion transport, downregulation of anion transport, inhibition of anion transport Relationships: is a type of GO:0043271; is a type of regulation of monoatomic anion transport [GO:0044070]; negatively regulates GO:0006820 Definition: Any process that stops, prevents or reduces the frequency, rate or extent of anion transport.